{
  "term_label": "Unknown biological process",
  "gene_name": "Polyadenylate-binding protein 1",
  "gene": "UniProtKB:P11940",
  "term_id": "UNKNOWN:0002",
  "gene_symbol": "PABPC1"
}